{
  "gene_name": "Zinc finger CW-type PWWP domain protein 2",
  "term_id": "UNKNOWN:0002",
  "term_label": "Unknown biological process",
  "gene": "UniProtKB:Q504Y3",
  "gene_symbol": "ZCWPW2"
}